regulation of calcium ion export across plasma membrane [GO:1905912] (biological process) Relationships: is a type of GO:1903169; regulates calcium ion export across plasma membrane [GO:1990034] Subtypes: GO:1905913, positive regulation of calcium ion export across plasma membrane [GO:1905914] References: PMID:22362515 Sources: GOC:BHF, GOC:BHF_miRNA, GOC:TermGenie, GOC:rph, GO_REF:0000058 Also known as: regulation of calcium ion efflux from cell, regulation of calcium ion export from cell Definition: Any process that modulates the frequency, rate or extent of calcium ion export across the plasma membrane.